asioloorosomucoid beta-1,3-glucuronosyltransferase activity [GO:0046988] (molecular function) Definition: Catalysis of the transfer, in a beta 1,3 linkage, of D-glucuronic acid (GlcUA) from UDP-GlcUA to asioloorosomucoid. Relationships: is a type of glucuronosyltransferase activity [GO:0015020] References: PMID:12511570 Sources: GOC:bf